{
  "gene": "UniProtKB:Q8TBZ0",
  "term_label": "Unknown biological process",
  "term_id": "UNKNOWN:0002",
  "gene_symbol": "CCDC110",
  "gene_name": "Coiled-coil domain-containing protein 110"
}